regulation of asexual sporulation resulting in formation of a cellular spore [GO:0043943] (biological process) Subtypes: GO:0043944, GO:0043945, regulation of aeciospore formation [GO:0075248], regulation of uredospore formation [GO:0075252], regulation of teliospore formation [GO:0075256], regulation of sporangiospore formation [GO:0075286] Definition: Any process that modulates the frequency, rate or extent of the formation of a cellular spore derived from the products of mitosis. Relationships: is a type of GO:0034305; is a type of regulation of sporulation resulting in formation of a cellular spore [GO:0042173]; regulates asexual sporulation resulting in formation of a cellular spore [GO:0043936] Sources: GOC:pamgo_curators